{
  "gene": "UniProtKB:Q9H0J9",
  "term_id": "GO:0003950",
  "gene_name": "Protein mono-ADP-ribosyltransferase PARP12",
  "gene_symbol": "PARP12",
  "term_label": "NAD+ poly-ADP-ribosyltransferase activity"
}